{
  "gene": "UniProtKB:Q6UXK2",
  "gene_name": "Immunoglobulin superfamily containing leucine-rich repeat protein 2",
  "gene_symbol": "ISLR2",
  "term_id": "GO:0009986",
  "term_label": "cell surface"
}